cytoskeleton-nuclear membrane anchor activity [GO:0140444] (molecular function) Also known as: cytoskeletal protein-nuclear membrane adaptor activity, cytoskeletal protein-nuclear membrane anchor activity, cytoskeleton nuclear membrane anchor activity, nuclear membrane-cytoskeleton anchor activity Relationships: is a type of GO:0043495 References: PMID:16237665 Definition: The binding activity of a molecule that brings together a cytoskeletal protein or protein complex and a nuclear membrane lipid or membrane-associated protein, in order to maintain the localization of the cytoskeleton at a specific location of the nuclear membrane.